{
  "gene_name": "Cryptic protein",
  "term_label": "activin receptor binding",
  "term_id": "GO:0070697",
  "gene_symbol": "CFC1",
  "gene": "UniProtKB:P0CG37"
}